{
  "gene_symbol": "RP2",
  "term_label": "GTPase activator activity",
  "gene_name": "Protein XRP2",
  "term_id": "GO:0005096",
  "gene": "UniProtKB:O75695"
}